{
  "gene_name": "Na(+)_H(+) exchange regulatory cofactor NHE-RF2",
  "gene": "UniProtKB:Q15599",
  "term_id": "GO:0005102",
  "term_label": "signaling receptor binding",
  "gene_symbol": "NHERF2"
}